{
  "gene_name": "Thioredoxin domain-containing protein 2",
  "term_id": "UNKNOWN:0003",
  "gene": "UniProtKB:Q86VQ3",
  "term_label": "Unknown cellular component",
  "gene_symbol": "TXNDC2"
}